{
  "term_id": "UNKNOWN:0002",
  "gene_symbol": "LINC02914",
  "term_label": "Unknown biological process",
  "gene": "UniProtKB:Q52M58",
  "gene_name": "Testis-specific protein LINC02914"
}